{
  "gene_symbol": "UBE2D4",
  "gene_name": "Ubiquitin-conjugating enzyme E2 D4",
  "term_id": "GO:0005634",
  "term_label": "nucleus",
  "gene": "UniProtKB:Q9Y2X8"
}